{
  "gene_symbol": "HMGA2",
  "term_label": "minor groove of adenine-thymine-rich DNA binding",
  "term_id": "GO:0003680",
  "gene_name": "High mobility group protein HMGI-C",
  "gene": "UniProtKB:P52926"
}